{
  "gene_symbol": "AAGAB",
  "term_label": "Unknown molecular function",
  "gene": "UniProtKB:Q6PD74",
  "term_id": "UNKNOWN:0001",
  "gene_name": "Alpha- and gamma-adaptin-binding protein p34"
}